{
  "gene": "UniProtKB:Q9NS61",
  "term_label": "regulation of signal transduction",
  "gene_name": "Kv channel-interacting protein 2",
  "term_id": "GO:0009966",
  "gene_symbol": "KCNIP2"
}